{
  "term_id": "GO:0051015",
  "gene_symbol": "IQGAP3",
  "term_label": "actin filament binding",
  "gene_name": "Ras GTPase-activating-like protein IQGAP3",
  "gene": "UniProtKB:Q86VI3"
}